{
  "term_label": "NADPH oxidase complex",
  "gene_symbol": "NOX5",
  "term_id": "GO:0043020",
  "gene_name": "NADPH oxidase 5",
  "gene": "UniProtKB:Q96PH1"
}